{
  "gene": "UniProtKB:Q9BZH6",
  "gene_symbol": "WDR11",
  "term_label": "Unknown biological process",
  "gene_name": "WD repeat-containing protein 11",
  "term_id": "UNKNOWN:0002"
}